{
  "gene_symbol": "EXOSC4",
  "gene": "UniProtKB:Q9NPD3",
  "gene_name": "Exosome complex component RRP41",
  "term_id": "GO:0000176",
  "term_label": "nuclear exosome (RNase complex)"
}